{
  "term_id": "UNKNOWN:0003",
  "term_label": "Unknown cellular component",
  "gene_symbol": "PRR15",
  "gene": "UniProtKB:Q8IV56",
  "gene_name": "Proline-rich protein 15"
}